{
  "term_id": "GO:0005868",
  "gene": "UniProtKB:Q8NCM8",
  "gene_symbol": "DYNC2H1",
  "term_label": "cytoplasmic dynein complex",
  "gene_name": "Cytoplasmic dynein 2 heavy chain 1"
}